{
  "term_id": "GO:0005743",
  "gene": "UniProtKB:Q9Y276",
  "gene_name": "Mitochondrial chaperone BCS1",
  "gene_symbol": "BCS1L",
  "term_label": "mitochondrial inner membrane"
}